regulation of intracellular pH [GO:0051453] (biological process) Subtypes: regulation of cellular pH reduction [GO:0032847], regulation of lysosomal lumen pH [GO:0035751], intracellular pH reduction [GO:0051452], intracellular pH elevation [GO:0051454] Definition: Any process that modulates the internal pH of a cell, measured by the concentration of the hydrogen ion. Relationships: is a type of GO:0030641; is a type of regulation of biological quality [GO:0065008] Sources: GOC:ai, GOC:dph, GOC:tb Also known as: cell pH regulation, cellular pH regulation, pH regulation in cell, regulation of cell pH